{
  "gene_name": "Olfactory receptor 5D14",
  "term_id": "GO:0007608",
  "gene": "UniProtKB:Q8NGL3",
  "gene_symbol": "OR5D14",
  "term_label": "sensory perception of smell"
}